{
  "term_id": "GO:0010507",
  "gene": "UniProtKB:P51397",
  "term_label": "negative regulation of autophagy",
  "gene_name": "Death-associated protein 1",
  "gene_symbol": "DAP"
}